{
  "term_label": "nucleus",
  "gene": "UniProtKB:A6NC97",
  "gene_name": "Putative protein FAM172B",
  "term_id": "GO:0005634",
  "gene_symbol": "ARB2BP"
}